{
  "gene_name": "La-related protein 6",
  "term_label": "Unknown biological process",
  "gene_symbol": "LARP6",
  "term_id": "UNKNOWN:0002",
  "gene": "UniProtKB:Q9BRS8"
}